{
  "term_label": "ferric iron binding",
  "gene": "UniProtKB:Q9BXU8",
  "gene_name": "Ferritin heavy polypeptide-like 17",
  "term_id": "GO:0008199",
  "gene_symbol": "FTHL17"
}